{
  "term_label": "actin filament-based movement",
  "gene_name": "Unconventional myosin-Ih",
  "gene": "UniProtKB:Q8N1T3",
  "gene_symbol": "MYO1H",
  "term_id": "GO:0030048"
}